G2 phase [GO:0051319] (biological process) Subtypes: GO:0000085, meiotic G2 phase [GO:0051331] Sources: GOC:mtg_cell_cycle Note: Note that this term should not be used for direct annotation. If you are trying to make an annotation to x phase, it is likely that the correct annotation is 'regulation of x/y phase transition' or to a process which occurs during the reported phase (i.e mitotic DNA replication for mitotic S-phase). To capture the phase when a specific location or process is observed, the phase term can be used in an annotation extension (PMID:24885854) applied to a cellular component term (with the relation exists_during) or a biological process term (with the relation happens_during). Definition: The cell cycle 'gap' phase which is the interval between the completion of DNA synthesis and the beginning of DNA segregation (usually by mitosis or meiosis). Relationships: is_a GO:0022403; is part of interphase [GO:0051325]